{
  "gene_symbol": "STING1",
  "gene_name": "Stimulator of interferon genes protein",
  "term_label": "autophagosome assembly",
  "term_id": "GO:0000045",
  "gene": "UniProtKB:Q86WV6"
}